{
  "gene": "UniProtKB:Q8N2C3",
  "term_id": "UNKNOWN:0002",
  "gene_symbol": "DEPDC4",
  "term_label": "Unknown biological process",
  "gene_name": "DEP domain-containing protein 4"
}